troponin I binding [GO:0031013] (molecular function) Relationships: is a type of cytoskeletal protein binding [GO:0008092] Sources: GOC:mah, ISBN:0815316194 Definition: Binding to troponin I, the inhibitory subunit of the troponin complex.